{
  "gene_symbol": "SEMA3G",
  "term_id": "GO:0005886",
  "gene_name": "Semaphorin-3G",
  "term_label": "plasma membrane",
  "gene": "UniProtKB:Q9NS98"
}